{
  "term_label": "transcription preinitiation complex",
  "gene": "UniProtKB:Q00403",
  "term_id": "GO:0097550",
  "gene_symbol": "GTF2B",
  "gene_name": "Transcription initiation factor IIB"
}